cellular response to arsenite(3-) [GO:1903841] (BP) Definition: Any process that results in a change in state or activity of a cell (in terms of movement, secretion, enzyme production, gene expression, etc.) as a result of an arsenite(3-) stimulus. Relationships: is a type of GO:0071243; is a type of GO:1901701; is a type of response to arsenite(3-) [GO:1903840] References: PMID:12106899 Sources: GOC:TermGenie, GOC:mr, GO_REF:0000071